{
  "gene_symbol": "VGLL1",
  "term_id": "GO:0005634",
  "gene_name": "Transcription cofactor vestigial-like protein 1",
  "term_label": "nucleus",
  "gene": "UniProtKB:Q99990"
}